{
  "gene_symbol": "RNF212",
  "gene_name": "Probable E3 SUMO-protein ligase RNF212",
  "gene": "UniProtKB:Q495C1",
  "term_label": "SUMO transferase activity",
  "term_id": "GO:0019789"
}